{
  "term_label": "negative regulation of membrane protein ectodomain proteolysis",
  "gene_symbol": "TIMP4",
  "gene": "UniProtKB:Q99727",
  "gene_name": "Metalloproteinase inhibitor 4",
  "term_id": "GO:0051045"
}